{
  "gene_name": "Ciliogenesis and planar polarity effector 2",
  "gene_symbol": "CPLANE2",
  "term_id": "GO:0005814",
  "gene": "UniProtKB:Q9BU20",
  "term_label": "centriole"
}